{
  "gene": "UniProtKB:Q92796",
  "term_id": "GO:0035255",
  "gene_name": "Disks large homolog 3",
  "gene_symbol": "DLG3",
  "term_label": "ionotropic glutamate receptor binding"
}